{
  "term_label": "Unknown molecular function",
  "gene_symbol": "ZNF436-AS1",
  "term_id": "UNKNOWN:0001",
  "gene": "UniProtKB:Q8NC38",
  "gene_name": "Putative uncharacterized protein ZNF436-AS1"
}